purine deoxyribonucleoside catabolic process [GO:0046124] (BP) Relationships: is a type of purine nucleoside catabolic process [GO:0006152]; is a type of deoxyribonucleoside catabolic process [GO:0046121]; is a type of purine deoxyribonucleoside metabolic process [GO:0046122] Also known as: purine deoxyribonucleoside breakdown, purine deoxyribonucleoside catabolism, purine deoxyribonucleoside degradation Definition: The chemical reactions and pathways resulting in the breakdown of any one of a family of organic molecules consisting of a purine base covalently bonded to a sugar deoxyribose (a deoxyribonucleoside). Sources: GOC:ai Subtypes: deoxyinosine catabolic process [GO:0006149], GO:0006157, GO:0006161